catagen [GO:0042637] (biological process) Definition: The regression phase of the hair cycle during which cell proliferation ceases, the hair follicle shortens, and an anchored club hair is produced. Regulation: regulated by GO:0051794; positively regulated by GO:0051795; negatively regulated by negative regulation of timing of catagen [GO:0051796] Also known as: hair regression References: PMID:12535193 Note: Note that this term should not be used for direct annotation. If you are trying to make an annotation to x phase, it is likely that the correct annotation is 'regulation of x/y phase transition' or to a process which occurs during the reported phase. To capture the phase when a specific location or process is observed, the phase term can be used in an annotation extension (PMID:24885854) applied to a cellular component term (with the relation exists_during) or a biological process term (with the relation happens_during). Relationships: is a type of hair cycle phase [GO:0044851]; is part of hair follicle maturation [GO:0048820]